{
  "term_id": "GO:0005868",
  "gene_symbol": "DYNLT2B",
  "term_label": "cytoplasmic dynein complex",
  "gene_name": "Dynein light chain Tctex-type protein 2B",
  "gene": "UniProtKB:Q8WW35"
}